{
  "term_label": "cytoplasm",
  "gene_symbol": "BMP2K",
  "gene_name": "BMP-2-inducible protein kinase",
  "gene": "UniProtKB:Q9NSY1",
  "term_id": "GO:0005737"
}